{
  "gene_symbol": "SIRT7",
  "gene_name": "NAD-dependent protein deacetylase sirtuin-7",
  "term_id": "GO:0097372",
  "gene": "UniProtKB:Q9NRC8",
  "term_label": "histone H3K18 deacetylase activity, NAD-dependent"
}